negative regulation of protein targeting to vacuole involved in autophagy [GO:1904052] (biological process) Also known as: down regulation of protein targeting to vacuole involved in autophagy, down-regulation of protein targeting to vacuole involved in autophagy, downregulation of protein targeting to vacuole involved in autophagy, inhibition of protein targeting to vacuole involved in autophagy Note: An example of this is SMURF1 in human (UniProt symbol Q9HCE7) in PMID:22020285 (inferred from mutant phenotype). Relationships: is a type of negative regulation of intracellular protein transport [GO:0090317]; is a type of negative regulation of vacuolar transport [GO:1903336]; is a type of regulation of protein targeting to vacuole involved in autophagy [GO:1904051]; RO_0002212 protein targeting to vacuole involved in autophagy [GO:0071211] Definition: Any process that stops, prevents or reduces the frequency, rate or extent of protein targeting to vacuole involved in autophagy. References: PMID:22020285 Sources: GOC:PARL, GOC:TermGenie, GOC:pad, GO_REF:0000058